{
  "gene_name": "Phosphoglucomutase-like protein 5",
  "gene": "UniProtKB:Q15124",
  "term_label": "sarcolemma",
  "term_id": "GO:0042383",
  "gene_symbol": "PGM5"
}